growth hormone-releasing hormone receptor binding [GO:0031770] (molecular function) Definition: Binding to a growth hormone-releasing hormone receptor. Sources: GOC:mah, GOC:nln Relationships: is a type of neuropeptide receptor binding [GO:0071855] Also known as: growth hormone-releasing hormone receptor ligand